{
  "term_label": "lysosome",
  "gene_name": "Ras-related protein Rab-7a",
  "gene": "UniProtKB:P51149",
  "gene_symbol": "RAB7A",
  "term_id": "GO:0005764"
}